regulation of alpha-beta T cell differentiation [GO:0046637] (biological process) Relationships: is a type of regulation of T cell differentiation [GO:0045580]; is a type of regulation of alpha-beta T cell activation [GO:0046634]; regulates alpha-beta T cell differentiation [GO:0046632] Subtypes: regulation of CD4-positive, alpha-beta T cell differentiation [GO:0043370], regulation of CD8-positive, alpha-beta T cell differentiation [GO:0043376], GO:0046638, GO:0046639, regulation of NK T cell differentiation [GO:0051136] Also known as: regulation of alpha-beta T lymphocyte differentiation, regulation of alpha-beta T-cell differentiation, regulation of alpha-beta T-lymphocyte differentiation, regulation of alpha-beta T cell development Definition: Any process that modulates the frequency, rate or extent of alpha-beta T cell differentiation. Note: Note that immunologists typically use the word 'development' to refer to cells of B or T cell lineages undergoing the process that GO describes as 'cell differentiation'. Sources: GOC:ai